sulfoacetaldehyde dehydrogenase activity [GO:0102984] (molecular function) Definition: Catalysis of the reaction: sulfonatoacetaldehyde + H2O + NAD = sulfonatoacetate + NADH + 2 H+. Sources: EC:1.2.1.73, GOC:pz Relationships: is a type of oxidoreductase activity, acting on the aldehyde or oxo group of donors, NAD or NADP as acceptor [GO:0016620]